{
  "term_label": "extracellular space",
  "gene_symbol": "TIMP1",
  "term_id": "GO:0005615",
  "gene": "UniProtKB:P01033",
  "gene_name": "Metalloproteinase inhibitor 1"
}